{
  "term_label": "cysteine-type deubiquitinase activity",
  "gene_symbol": "USP37",
  "term_id": "GO:0004843",
  "gene": "UniProtKB:Q86T82",
  "gene_name": "Ubiquitin carboxyl-terminal hydrolase 37"
}